{
  "term_label": "mitochondrial large ribosomal subunit",
  "gene_name": "Large ribosomal subunit protein bL34m",
  "term_id": "GO:0005762",
  "gene": "UniProtKB:Q9BQ48",
  "gene_symbol": "MRPL34"
}